carbon catabolite repression of transcription [GO:0045013] (BP) Subtypes: carbon catabolite repression of transcription by galactose [GO:0000410], carbon catabolite repression of transcription from RNA polymerase II promoter [GO:0000437], carbon catabolite repression of transcription by glucose [GO:0045014] Also known as: negative regulation of transcription by carbon catabolites, carbon catabolite repression Relationships: is a type of GO:0045892; is a type of GO:0045990; is_a carbon catabolite repression [GO:0061985] Definition: A transcription regulation process in which the presence of one carbon source leads to a decrease in the frequency, rate, or extent of transcription of specific genes involved in the metabolism of other carbon sources. Carbon catabolite repression is a mechanism of genetic regulation which the accumulation of catabolites of one substance in the cell represses the formation of enzymes that contribute to the catabolism of other substances. References: PMID:11018147, PMID:18359269, PMID:9618445 Sources: GOC:mah, ISBN:0198506732